{
  "gene_name": "Putative solute carrier family 26 member 10P",
  "gene_symbol": "SLC26A10P",
  "term_label": "chloride transmembrane transport",
  "term_id": "GO:1902476",
  "gene": "UniProtKB:Q8NG04"
}